{
  "gene_name": "Stabilin-2",
  "term_label": "low-density lipoprotein particle binding",
  "term_id": "GO:0030169",
  "gene_symbol": "STAB2",
  "gene": "UniProtKB:Q8WWQ8"
}